adenine salvage [GO:0006168] (biological process) Also known as: adenine, hypoxanthine and their nucleoside salvage, adenine salvage pathway Definition: Any process that generates adenine, 6-aminopurine, from derivatives of it without de novo synthesis. Sources: GOC:jl Relationships: is a type of purine nucleobase salvage [GO:0043096]; is a type of adenine biosynthetic process [GO:0046084]